{
  "term_id": "GO:0004843",
  "gene_name": "Ubiquitin carboxyl-terminal hydrolase 17-like protein 3",
  "term_label": "cysteine-type deubiquitinase activity",
  "gene": "UniProtKB:A6NCW0",
  "gene_symbol": "USP17L3"
}